CD8-positive, alpha-beta intraepithelial T cell differentiation [GO:0002300] (biological process) Definition: The process in which a precursor cell type acquires the specialized features of a CD8-positive, alpha-beta intraepithelial T cell. Intraepithelial T cells are found among epithelial cells in mucosal areas and have distinct phenotypes and developmental pathways. Note: Note that immunologists typically use the word 'development' to refer to cells of B or T cell lineages undergoing the process that GO describes as 'cell differentiation'. Also known as: CD8-positive, alpha-beta intraepithelial T lymphocyte differentiation, CD8-positive, alpha-beta intraepithelial T-cell differentiation, CD8-positive, alpha-beta intraepithelial T-lymphocyte differentiation, CD8-positive, alpha-beta intraepithelial T cell development Sources: GOC:add, ISBN:0781735149 Relationships: is a type of alpha-beta intraepithelial T cell differentiation [GO:0002299]; is a type of CD8-positive, alpha-beta T cell differentiation [GO:0043374]